tetraterpenoid transport [GO:0046866] (biological process) Sources: GOC:ai Definition: The directed movement of tetraterpenoids into, out of or within a cell, or between cells, by means of some agent such as a transporter or pore. Tetraterpenoids are terpenoids with eight isoprene units. Subtypes: GO:0046867 Relationships: is_a terpenoid transport [GO:0046865]